gallate catabolic process via 2-pyrone-4,6-dicarboxylate [GO:0019397] (biological process) Sources: GOC:jl Also known as: gallate breakdown via 2-pyrone-4,6-dicarboxylate, gallate degradation via 2-pyrone-4,6-dicarboxylate, gallic acid catabolic process via 2-pyrone-4,6-dicarboxylate, gallic acid catabolism via 2-pyrone-4,6-dicarboxylate Definition: The chemical reactions and pathways resulting in the breakdown of gallate, the anion of gallic acid, via the intermediate 2-pyrone-4,6-dicarboxylate. Relationships: is_a aerobic gallate catabolic process [GO:0042195]